{
  "gene_name": "Phosphatidylcholine transfer protein",
  "gene_symbol": "PCTP",
  "term_id": "GO:0008525",
  "gene": "UniProtKB:Q9UKL6",
  "term_label": "phosphatidylcholine transporter activity"
}